{
  "term_label": "Unknown molecular function",
  "term_id": "UNKNOWN:0001",
  "gene_name": "tRNA endonuclease ANKZF1",
  "gene": "UniProtKB:Q9H8Y5",
  "gene_symbol": "ANKZF1"
}